{
  "term_id": "GO:0006531",
  "gene_name": "D-aspartate oxidase",
  "gene_symbol": "DDO",
  "gene": "UniProtKB:Q99489",
  "term_label": "aspartate metabolic process"
}